maltopentaose transport [GO:2001101] (biological process) Sources: GOC:mengo_curators Relationships: is a type of pentasaccharide transport [GO:2001100] Regulation: regulated by regulation of maltopentaose transport [GO:1900315]; negatively regulated by GO:1900316; positively regulated by GO:1900317 Definition: The directed movement of a maltopentaoseacetate into, out of or within a cell, or between cells, by means of some agent such as a transporter or pore.